{
  "term_label": "response to estradiol",
  "term_id": "GO:0032355",
  "gene_symbol": "CYP19A1",
  "gene_name": "Aromatase",
  "gene": "UniProtKB:P11511"
}